{
  "term_label": "Unknown molecular function",
  "gene_symbol": "TNKS1BP1",
  "term_id": "UNKNOWN:0001",
  "gene": "UniProtKB:Q9C0C2",
  "gene_name": "182 kDa tankyrase-1-binding protein"
}